{
  "gene_name": "Protein ILRUN",
  "term_id": "GO:0043130",
  "gene_symbol": "ILRUN",
  "term_label": "ubiquitin binding",
  "gene": "UniProtKB:Q9H6K1"
}